{
  "gene_symbol": "G6PC2",
  "term_label": "glucose 6-phosphate metabolic process",
  "term_id": "GO:0051156",
  "gene": "UniProtKB:Q9NQR9",
  "gene_name": "Glucose-6-phosphatase 2"
}